{
  "term_id": "GO:0016477",
  "gene": "UniProtKB:P05106",
  "term_label": "cell migration",
  "gene_symbol": "ITGB3",
  "gene_name": "Integrin beta-3"
}